positive regulation of tRNA export from nucleus [GO:2000240] (biological process) Also known as: positive regulation of tRNA export from cell nucleus, positive regulation of tRNA export out of nucleus, positive regulation of tRNA transport from nucleus to cytoplasm, positive regulation of tRNA-nucleus export Relationships: is a type of GO:0046833; is a type of GO:2000199; is a type of GO:2000238; positively regulates tRNA export from nucleus [GO:0006409] Sources: GOC:mah Definition: Any process that activates or increases the frequency, rate or extent of tRNA export from nucleus.